{
  "gene_symbol": "CDK15",
  "gene_name": "Cyclin-dependent kinase 15",
  "term_label": "cyclin binding",
  "term_id": "GO:0030332",
  "gene": "UniProtKB:Q96Q40"
}